{
  "gene_name": "Medium-chain specific acyl-CoA dehydrogenase, mitochondrial",
  "gene": "UniProtKB:P11310",
  "term_label": "mitochondrion",
  "gene_symbol": "ACADM",
  "term_id": "GO:0005739"
}